{
  "term_label": "negative regulation of transcription by RNA polymerase II",
  "gene": "UniProtKB:Q9UBC3",
  "gene_name": "DNA (cytosine-5)-methyltransferase 3B",
  "term_id": "GO:0000122",
  "gene_symbol": "DNMT3B"
}